{
  "gene": "UniProtKB:Q6UWB1",
  "term_label": "interleukin-27 receptor activity",
  "gene_symbol": "IL27RA",
  "gene_name": "Interleukin-27 receptor subunit alpha",
  "term_id": "GO:0045509"
}